carbohydrate storage [GO:0052576] (biological process) Definition: The accumulation and maintenance in cells or tissues of carbohydrates, any of a group of organic compounds based of the general formula Cx(H2O)y. Relationships: is a type of GO:0052575 References: PMID:10758476